{
  "gene_name": "60 kDa heat shock protein, mitochondrial",
  "term_id": "GO:0050870",
  "gene_symbol": "HSPD1",
  "gene": "UniProtKB:P10809",
  "term_label": "positive regulation of T cell activation"
}